regulation of antisense RNA transcription [GO:0060194] (BP) References: PMID:18075583 Sources: GOC:dph, GOC:jp, GOC:tb Subtypes: negative regulation of antisense RNA transcription [GO:0060195], GO:0060196 Definition: Any process that modulates the frequency, rate or extent of the synthesis of antisense RNA, an RNA molecule complementary in sequence to another RNA or DNA molecule, which, by binding the latter, acts to inhibit its function and/or completion of synthesis, on a template of DNA. Relationships: is a type of GO:0006355; regulates GO:0009300